programmed cell death in response to retinoic acid [GO:0160059] (biological process) Also known as: retinoic acid-induced apoptosis References: PMID:17869331, PMID:9187263 Relationships: is a type of GO:0012501; is part of GO:0071300 Definition: Cell death resulting from activation of endogenous cellular processes and occurring as a result of a retinoic acid.